{
  "term_label": "cytoplasm",
  "gene": "UniProtKB:P57058",
  "gene_symbol": "HUNK",
  "term_id": "GO:0005737",
  "gene_name": "Hormonally up-regulated neu tumor-associated kinase"
}